{
  "gene": "UniProtKB:P13762",
  "gene_symbol": "HLA-DRB4",
  "gene_name": "HLA class II histocompatibility antigen, DR beta 4 chain",
  "term_id": "GO:0019886",
  "term_label": "antigen processing and presentation of exogenous peptide antigen via MHC class II"
}